{
  "gene_symbol": "EIF2S3B",
  "term_id": "GO:0003743",
  "term_label": "translation initiation factor activity",
  "gene": "UniProtKB:Q2VIR3",
  "gene_name": "Eukaryotic translation initiation factor 2 subunit 3B"
}